{
  "term_label": "regulation of DNA-templated transcription",
  "gene_name": "Zinc finger protein 221",
  "gene": "UniProtKB:Q9UK13",
  "gene_symbol": "ZNF221",
  "term_id": "GO:0006355"
}